{
  "gene_symbol": "SRL",
  "gene_name": "Sarcalumenin",
  "term_id": "UNKNOWN:0001",
  "gene": "UniProtKB:Q86TD4",
  "term_label": "Unknown molecular function"
}